{
  "gene_name": "WW domain-containing transcription regulator protein 1",
  "term_id": "GO:0003714",
  "gene": "UniProtKB:Q9GZV5",
  "gene_symbol": "WWTR1",
  "term_label": "transcription corepressor activity"
}